{
  "gene": "UniProtKB:P20336",
  "gene_symbol": "RAB3A",
  "term_label": "plasma membrane",
  "term_id": "GO:0005886",
  "gene_name": "Ras-related protein Rab-3A"
}